{
  "gene": "UniProtKB:P33261",
  "gene_name": "Cytochrome P450 2C19",
  "gene_symbol": "CYP2C19",
  "term_id": "GO:0020037",
  "term_label": "heme binding"
}